{
  "gene_symbol": "PLCXD1",
  "gene": "UniProtKB:Q9NUJ7",
  "term_id": "UNKNOWN:0002",
  "gene_name": "PI-PLC X domain-containing protein 1",
  "term_label": "Unknown biological process"
}